Doa10p ubiquitin ligase complex [GO:0000837] (cellular component) Also known as: Ssm4p ubiquitin ligase complex References: PMID:16873066 Sources: GOC:elh Relationships: is a type of ER ubiquitin ligase complex [GO:0000835] Definition: A multiprotein complex that recognizes and ubiquitinates membrane proteins with misfolded cytosolic domains during ER-associated protein degradation (ERAD). In S. cerevisiae, this complex contains the ubiquitin ligase Ssm4p/Doa10p.